{
  "term_label": "microtubule-based movement",
  "term_id": "GO:0007018",
  "gene": "UniProtKB:Q9HAQ2",
  "gene_symbol": "KIF9",
  "gene_name": "Kinesin-like protein KIF9"
}